{
  "gene": "UniProtKB:Q9Y303",
  "term_label": "Unknown cellular component",
  "gene_symbol": "AMDHD2",
  "term_id": "UNKNOWN:0003",
  "gene_name": "N-acetylglucosamine-6-phosphate deacetylase"
}